outer mucus layer [GO:0070703] (cellular component) References: PMID:18806221, PMID:19432394 Sources: GOC:mah, GOC:mm2 Definition: The outer of two mucus layers secreted by epithelial cells in the colon; the outer mucus layer is loosely packed and can be colonized by bacteria. Relationships: is a type of mucus layer [GO:0070701]